{
  "gene": "UniProtKB:P55291",
  "term_id": "GO:0007043",
  "term_label": "cell-cell junction assembly",
  "gene_name": "Cadherin-15",
  "gene_symbol": "CDH15"
}